cell wall polysaccharide metabolic process [GO:0010383] (biological process) Definition: The chemical reactions and pathways involving cell wall polysaccharides. Relationships: is a type of polysaccharide metabolic process [GO:0005976]; is a type of cell wall macromolecule metabolic process [GO:0044036] Subtypes: rhamnogalacturonan I metabolic process [GO:0010395], mannan metabolic process [GO:0010412], cell wall beta-glucan metabolic process [GO:0034406], GO:0044347, GO:0070592, cell wall (1->3)-alpha-glucan metabolic process [GO:0070597], GO:0071966 Sources: GOC:tair_curators